{
  "term_label": "brain development",
  "term_id": "GO:0007420",
  "gene_symbol": "SOX21",
  "gene": "UniProtKB:Q9Y651",
  "gene_name": "Transcription factor SOX-21"
}